{
  "gene_symbol": "CCNA2",
  "term_label": "nucleus",
  "gene": "UniProtKB:P20248",
  "term_id": "GO:0005634",
  "gene_name": "Cyclin-A2"
}